{
  "gene_name": "Neurotrophin-4",
  "term_label": "neuron projection morphogenesis",
  "gene_symbol": "NTF4",
  "term_id": "GO:0048812",
  "gene": "UniProtKB:P34130"
}